{
  "term_id": "GO:0000978",
  "gene_symbol": "ZNF253",
  "gene": "UniProtKB:O75346",
  "gene_name": "Zinc finger protein 253",
  "term_label": "RNA polymerase II cis-regulatory region sequence-specific DNA binding"
}